{
  "gene": "UniProtKB:P16220",
  "term_label": "regulation of transcription by RNA polymerase II",
  "term_id": "GO:0006357",
  "gene_symbol": "CREB1",
  "gene_name": "Cyclic AMP-responsive element-binding protein 1"
}